histone isonicotinyllysine deisonicotinylase activity [GO:0140229] (molecular function) Definition: Catalysis of the reaction: N(6)-isonicotinyl-L-lysyl-[protein] + H2O = isonicotinate + L-lysyl-[protein]. References: PMID:34545082 Relationships: is a type of histone modifying activity [GO:0140993]